{
  "gene_symbol": "RHOU",
  "term_label": "protein kinase binding",
  "gene": "UniProtKB:Q7L0Q8",
  "gene_name": "Rho-related GTP-binding protein RhoU",
  "term_id": "GO:0019901"
}